{
  "term_id": "GO:0016020",
  "gene": "UniProtKB:Q8NGY2",
  "gene_name": "Olfactory receptor 6K2",
  "gene_symbol": "OR6K2",
  "term_label": "membrane"
}